{
  "gene": "UniProtKB:O75179",
  "term_label": "cytoplasm",
  "term_id": "GO:0005737",
  "gene_symbol": "ANKRD17",
  "gene_name": "Ankyrin repeat domain-containing protein 17"
}